{
  "gene_name": "Alpha-ketoglutarate-dependent dioxygenase alkB homolog 3",
  "gene_symbol": "ALKBH3",
  "gene": "UniProtKB:Q96Q83",
  "term_label": "DNA repair",
  "term_id": "GO:0006281"
}